{
  "term_id": "UNKNOWN:0001",
  "gene_name": "Actin-related protein 3C",
  "term_label": "Unknown molecular function",
  "gene": "UniProtKB:Q9C0K3",
  "gene_symbol": "ACTR3C"
}